{
  "term_label": "JNK cascade",
  "gene_symbol": "MAPK9",
  "term_id": "GO:0007254",
  "gene": "UniProtKB:P45984",
  "gene_name": "Mitogen-activated protein kinase 9"
}